{
  "gene": "UniProtKB:P25874",
  "gene_symbol": "UCP1",
  "term_id": "GO:1990542",
  "term_label": "mitochondrial transmembrane transport",
  "gene_name": "Mitochondrial brown fat uncoupling protein 1"
}